{
  "gene_name": "Interferon-induced protein with tetratricopeptide repeats 1",
  "term_label": "cytosol",
  "gene_symbol": "IFIT1",
  "term_id": "GO:0005829",
  "gene": "UniProtKB:P09914"
}